neurofilament [GO:0005883] (cellular component) Relationships: is a type of intermediate filament [GO:0005882]; is part of cytoplasm [GO:0005737] Sources: ISBN:0198506732, ISBN:0716731363, ISBN:0815316194 Also known as: type IV intermediate filament Definition: A type of intermediate filament found in the core of neuronal axons. Neurofilaments are heteropolymers composed of three type IV polypeptides: NF-L, NF-M, and NF-H (for low, middle, and high molecular weight). Neurofilaments are responsible for the radial growth of an axon and determine axonal diameter.